syn-pimara-7,15-diene synthase activity [GO:0034279] (molecular function) Also known as: 9alpha-copalyl-diphosphate diphosphate-lyase (9beta-pimara-7,15-diene-forming) activity Sources: RHEA:25560 Relationships: is_a carbon-oxygen lyase activity, acting on phosphates [GO:0016838] Definition: Catalysis of the reaction: 9-alpha-copalyl diphosphate = 9-beta-pimara-7,15-diene + diphosphate.